{
  "gene_symbol": "MOSMO",
  "term_id": "UNKNOWN:0001",
  "gene_name": "Modulator of smoothened protein",
  "gene": "UniProtKB:Q8NHV5",
  "term_label": "Unknown molecular function"
}